histamine secretion, neurotransmission [GO:0061538] (biological process) Definition: The controlled release of histamine by a cell, in which the histamine acts as a neurotransmitter. Sources: GOC:dph Relationships: is_a histamine secretion [GO:0001821]; is a type of GO:0007269; is a type of organic cation transport [GO:0015695]; is_a GO:0015801; is a type of L-amino acid transport [GO:0015807]